{
  "term_id": "GO:0030335",
  "term_label": "positive regulation of cell migration",
  "gene_symbol": "CCL19",
  "gene": "UniProtKB:Q99731",
  "gene_name": "C-C motif chemokine 19"
}